{
  "term_id": "GO:1990023",
  "term_label": "mitotic spindle midzone",
  "gene_name": "Kinesin-like protein KIF18B",
  "gene_symbol": "KIF18B",
  "gene": "UniProtKB:Q86Y91"
}